{
  "term_id": "GO:0035556",
  "gene_symbol": "NRG3",
  "gene_name": "Pro-neuregulin-3, membrane-bound isoform",
  "term_label": "intracellular signal transduction",
  "gene": "UniProtKB:P56975"
}